GGG codon-amino acid adaptor activity [GO:0033464] (MF) Sources: GOC:mah Note: Note that in the standard genetic code, GGG codes for glycine. Also known as: glycine tRNA Relationships: is a type of triplet codon-amino acid adaptor activity [GO:0030533] Definition: A triplet codon-amino acid adaptor activity that recognizes a GGG codon.